neurohypophysis formation [GO:0048849] (biological process) Relationships: is a type of anatomical structure formation involved in morphogenesis [GO:0048646]; is part of neurohypophysis morphogenesis [GO:0048848] Sources: GOC:cls, GOC:dgh, GOC:dph, GOC:jid Also known as: neurophysis biosynthesis, neurophysis formation, posterior pituitary biosynthesis, posterior pituitary formation, posterior pituitary gland biosynthesis, posterior pituitary gland formation Definition: The process that gives rise to neurohypophysis. This process pertains to the initial formation of a structure from unspecified parts. The neurohypophysis is the part of the pituitary gland that secretes hormones involved in blood pressure regulation.